exit of virus from host cell nucleus via nuclear envelope disassembly [GO:0039677] (biological process) Sources: VZ:2176 Definition: The directed movement of the viral genome or a viral particle out of the host cell nucleus that involves disruption of the nuclear membrane envelope by the virus. Also known as: exit of virus from host cell nucleus via nuclear envelope breakdown Relationships: is a type of GO:0039674; BFO_0000051 nuclear membrane disassembly [GO:0051081]